{
  "term_id": "UNKNOWN:0001",
  "gene": "UniProtKB:Q8IUC1",
  "gene_symbol": "KRTAP11-1",
  "gene_name": "Keratin-associated protein 11-1",
  "term_label": "Unknown molecular function"
}